nephron epithelium development [GO:0072009] (biological process) Subtypes: mesonephric nephron epithelium development [GO:0061241], glomerular epithelium development [GO:0072010], macula densa development [GO:0072024], short descending thin limb development [GO:0072063], long descending thin limb development [GO:0072064], early distal convoluted tubule development [GO:0072067], GO:0072068, nephron tubule development [GO:0072080], metanephric nephron epithelium development [GO:0072243] Definition: The process whose specific outcome is the progression of the nephron epithelium over time, from its formation to the mature structure. An epithelium is a tissue that covers the internal or external surfaces of an anatomical structure. The nephron epithelium is a tissue that covers the surface of a nephron. Sources: GOC:mtg_kidney_jan10 Relationships: is a type of kidney epithelium development [GO:0072073]; is part of GO:0072006